{
  "term_id": "GO:0004352",
  "term_label": "glutamate dehydrogenase (NAD+) activity",
  "gene_symbol": "GLUD2",
  "gene_name": "Glutamate dehydrogenase 2, mitochondrial",
  "gene": "UniProtKB:P49448"
}